{
  "term_label": "positive regulation of bone mineralization",
  "gene": "UniProtKB:Q4V9L6",
  "gene_name": "Transmembrane protein 119",
  "gene_symbol": "TMEM119",
  "term_id": "GO:0030501"
}